unsaturated fatty acid metabolic process [GO:0033559] (biological process) Relationships: is a type of fatty acid metabolic process [GO:0006631] Subtypes: GO:0006636, prostanoid metabolic process [GO:0006692], arachidonate metabolic process [GO:0019369], GO:0036109, GO:0043651, lipoxin A4 metabolic process [GO:2001302], lipoxin B4 metabolic process [GO:2001304] Also known as: unsaturated fatty acid metabolism Definition: The chemical reactions and pathways involving an unsaturated fatty acid, any fatty acid containing one or more double bonds between carbon atoms. Sources: GOC:mah